{
  "term_label": "ephrin receptor signaling pathway",
  "gene_name": "Ephrin-A4",
  "gene": "UniProtKB:P52798",
  "gene_symbol": "EFNA4",
  "term_id": "GO:0048013"
}